cytokinetic process [GO:0032506] (BP) Subtypes: GO:0000912, division septum site selection [GO:0000918], cytokinesis, division site positioning [GO:0007105], GO:0007107, regulation of actomyosin contractile ring contraction [GO:0031991], cleavage furrow formation [GO:0036089], cleavage furrow ingression [GO:0036090], contractile ring contraction [GO:0036213], cell septum assembly [GO:0090529], mitotic cytokinetic process [GO:1902410] Regulation: regulated by regulation of cytokinetic process [GO:0032954] Sources: GOC:bf, GOC:isa_complete, GOC:mah Relationships: is a type of GO:0022402; is part of cytokinesis [GO:0000910] Definition: A cellular process that is involved in cytokinesis (the division of the cytoplasm of a cell and its separation into two daughter cells).